{
  "term_id": "GO:0008081",
  "gene_symbol": "APEX2",
  "gene": "UniProtKB:Q9UBZ4",
  "term_label": "phosphoric diester hydrolase activity",
  "gene_name": "DNA-(apurinic or apyrimidinic site) endonuclease 2"
}